C-rich strand telomeric DNA binding [GO:0061730] (molecular function) Definition: Binding to C-rich, single-stranded, telomere-associated DNA. References: PMID:18329362 Sources: GOC:dph, GOC:kmv Relationships: is a type of single-stranded telomeric DNA binding [GO:0043047]